{
  "gene": "UniProtKB:Q8NCL8",
  "term_label": "Unknown molecular function",
  "gene_symbol": "TMEM116",
  "term_id": "UNKNOWN:0001",
  "gene_name": "Transmembrane protein 116"
}